eugenol metabolic process [GO:0042854] (biological process) Definition: The chemical reactions and pathways involving eugenol, a colorless, aromatic, liquid hydrocarbon (C10H12O2) found in clove oil. Subtypes: eugenol biosynthetic process [GO:0042855], eugenol catabolic process [GO:0042856] Sources: GOC:jl Relationships: is a type of phenylpropanoid metabolic process [GO:0009698]; is a type of phenol-containing compound metabolic process [GO:0018958]; is a type of GO:0042537; is a type of olefinic compound metabolic process [GO:0120254] Also known as: 4-allyl-2-methoxyphenol metabolic process, 4-allyl-2-methoxyphenol metabolism, eugenic acid metabolic process, eugenic acid metabolism, eugenol metabolism